{
  "gene": "UniProtKB:P56539",
  "gene_symbol": "CAV3",
  "gene_name": "Caveolin-3",
  "term_label": "molecular adaptor activity",
  "term_id": "GO:0060090"
}